{
  "term_id": "GO:0005737",
  "gene_name": "Zyxin",
  "gene": "UniProtKB:Q15942",
  "term_label": "cytoplasm",
  "gene_symbol": "ZYX"
}